{
  "gene_name": "Histone lysine demethylase PHF8",
  "gene_symbol": "PHF8",
  "gene": "UniProtKB:Q9UPP1",
  "term_id": "GO:0003712",
  "term_label": "transcription coregulator activity"
}